negative regulation of estrogen biosynthetic process [GO:1904077] (biological process) Definition: Any process that stops, prevents or reduces the frequency, rate or extent of estrogen biosynthetic process. Also known as: down regulation of estrogen anabolism, down regulation of estrogen biosynthesis, down regulation of estrogen biosynthetic process, down regulation of estrogen formation, down regulation of estrogen synthesis, down regulation of oestrogen biosynthesis, down regulation of oestrogen biosynthetic process, down-regulation of estrogen anabolism, down-regulation of estrogen biosynthesis, down-regulation of estrogen biosynthetic process, down-regulation of estrogen formation, down-regulation of estrogen synthesis, down-regulation of oestrogen biosynthesis, down-regulation of oestrogen biosynthetic process, downregulation of estrogen anabolism, downregulation of estrogen biosynthesis, downregulation of estrogen biosynthetic process, downregulation of estrogen formation, downregulation of estrogen synthesis, downregulation of oestrogen biosynthesis, downregulation of oestrogen biosynthetic process, negative regulation of estrogen anabolism, negative regulation of estrogen biosynthesis, negative regulation of estrogen formation, negative regulation of estrogen synthesis, negative regulation of oestrogen biosynthesis, negative regulation of oestrogen biosynthetic process, inhibition of estrogen anabolism, inhibition of estrogen biosynthesis, inhibition of estrogen biosynthetic process, inhibition of estrogen formation, inhibition of estrogen synthesis, inhibition of oestrogen biosynthesis, inhibition of oestrogen biosynthetic process References: PMID:24530842 Sources: GOC:TermGenie, GO_REF:0000058 Relationships: is a type of negative regulation of steroid biosynthetic process [GO:0010894]; is_a negative regulation of hormone biosynthetic process [GO:0032353]; is a type of regulation of estrogen biosynthetic process [GO:1904076]; negatively regulates estrogen biosynthetic process [GO:0006703]